{
  "gene": "UniProtKB:Q9Y4X5",
  "gene_name": "E3 ubiquitin-protein ligase ARIH1",
  "term_label": "cytoplasm",
  "gene_symbol": "ARIH1",
  "term_id": "GO:0005737"
}